channel inhibitor activity [GO:0016248] (molecular function) Sources: GOC:mah Subtypes: ion channel inhibitor activity [GO:0008200] Relationships: is a type of GO:0016247; is_a transporter inhibitor activity [GO:0141110]; negatively regulates channel activity [GO:0015267] Definition: Binds to and stops, prevents, or reduces the activity of a channel.